{
  "term_id": "GO:0071280",
  "gene_name": "Metallothionein-4",
  "gene_symbol": "MT4",
  "term_label": "cellular response to copper ion",
  "gene": "UniProtKB:P47944"
}